negative regulation of establishment of bipolar cell polarity [GO:1904846] (biological process) Definition: Any process that stops, prevents or reduces the frequency, rate or extent of establishment of bipolar cell polarity. References: PMID:26525038 Sources: GOC:TermGenie, GO_REF:0000058 Also known as: down regulation of establishment of bipolar cell polarity, down-regulation of establishment of bipolar cell polarity, downregulation of establishment of bipolar cell polarity, inhibition of establishment of bipolar cell polarity Relationships: is a type of GO:0048523; is a type of regulation of establishment of bipolar cell polarity [GO:0061172]; negatively regulates GO:0061171